{
  "gene": "UniProtKB:O14896",
  "gene_symbol": "IRF6",
  "term_id": "GO:0006357",
  "term_label": "regulation of transcription by RNA polymerase II",
  "gene_name": "Interferon regulatory factor 6"
}